{
  "term_label": "nerve growth factor signaling pathway",
  "term_id": "GO:0038180",
  "gene": "UniProtKB:P01138",
  "gene_symbol": "NGF",
  "gene_name": "Beta-nerve growth factor"
}